{
  "gene_name": "Putative serine_threonine-protein kinase SIK1B",
  "term_label": "Unknown cellular component",
  "gene_symbol": "SIK1B",
  "term_id": "UNKNOWN:0003",
  "gene": "UniProtKB:A0A0B4J2F2"
}